{
  "term_id": "GO:0098703",
  "gene": "UniProtKB:B1AL88",
  "gene_symbol": "NALF1",
  "term_label": "calcium ion import across plasma membrane",
  "gene_name": "NALCN channel auxiliary factor 1"
}